{
  "term_id": "GO:0005471",
  "gene_symbol": "SLC25A31",
  "gene": "UniProtKB:Q9H0C2",
  "gene_name": "ADP_ATP translocase 4",
  "term_label": "ATP:ADP antiporter activity"
}